serine racemase activity [GO:0030378] (molecular function) Relationships: is a type of GO:0047661 Definition: Catalysis of the reaction: L-serine = D-serine. Sources: RHEA:10980